{
  "term_id": "UNKNOWN:0001",
  "gene_symbol": "BCAS1",
  "gene": "UniProtKB:O75363",
  "term_label": "Unknown molecular function",
  "gene_name": "Breast carcinoma-amplified sequence 1"
}